{
  "gene_symbol": "SDHB",
  "gene_name": "Succinate dehydrogenase [ubiquinone] iron-sulfur subunit, mitochondrial",
  "term_id": "GO:0009060",
  "gene": "UniProtKB:P21912",
  "term_label": "aerobic respiration"
}